atrial septum intermedium morphogenesis [GO:0003291] (biological process) Sources: GOC:mtg_heart Definition: The process in which anatomical structure of an atrial septum intermedium is generated and organized. Relationships: is a type of atrial septum morphogenesis [GO:0060413]; is part of atrial septum intermedium development [GO:0003286]